positive regulation of interleukin-15 production [GO:0032738] (biological process) Definition: Any process that activates or increases the frequency, rate, or extent of interleukin-15 production. Sources: GOC:mah Also known as: positive regulation of IL-15 production, up regulation of interleukin-15 production, up-regulation of interleukin-15 production, upregulation of interleukin-15 production, activation of interleukin-15 production, positive regulation of interleukin-15 biosynthetic process, stimulation of interleukin-15 production Relationships: is a type of GO:0001819; is a type of regulation of interleukin-15 production [GO:0032658]; RO_0002213 GO:0032618